{
  "gene_symbol": "SIRT2",
  "term_label": "nucleus",
  "gene_name": "NAD-dependent protein deacetylase sirtuin-2",
  "term_id": "GO:0005634",
  "gene": "UniProtKB:Q8IXJ6"
}